midbody [GO:0030496] (cellular component) Sources: ISBN:0815316194 Relationships: is a type of cellular anatomical structure [GO:0110165] Definition: A thin cytoplasmic bridge formed between daughter cells at the end of cytokinesis. The midbody forms where the contractile ring constricts, and may persist for some time before finally breaking to complete cytokinesis.